{
  "gene_name": "Ret finger protein-like 2",
  "gene": "UniProtKB:O75678",
  "gene_symbol": "RFPL2",
  "term_label": "ubiquitin protein ligase activity",
  "term_id": "GO:0061630"
}